{
  "gene_name": "Myeloid zinc finger 1",
  "term_label": "RNA polymerase II cis-regulatory region sequence-specific DNA binding",
  "gene": "UniProtKB:P28698",
  "gene_symbol": "MZF1",
  "term_id": "GO:0000978"
}